{
  "term_label": "intracellular signal transduction",
  "term_id": "GO:0035556",
  "gene_name": "p53-induced death domain-containing protein 1",
  "gene": "UniProtKB:Q9HB75",
  "gene_symbol": "PIDD1"
}